{
  "term_label": "cell surface",
  "term_id": "GO:0009986",
  "gene_name": "Trem-like transcript 2 protein",
  "gene": "UniProtKB:Q5T2D2",
  "gene_symbol": "TREML2"
}